{
  "term_id": "GO:0006357",
  "gene": "UniProtKB:Q12824",
  "term_label": "regulation of transcription by RNA polymerase II",
  "gene_name": "SWI_SNF-related matrix-associated actin-dependent regulator of chromatin subfamily B member 1",
  "gene_symbol": "SMARCB1"
}